mesonephric glomerulus vasculature morphogenesis [GO:0061248] (biological process) Relationships: is a type of glomerulus vasculature morphogenesis [GO:0072103]; is part of mesonephric glomerulus vasculature development [GO:0061231]; is part of mesonephric glomerulus morphogenesis [GO:0061234] Definition: The process in which the anatomical structures of the mesonephric glomerulus vasculature are generated and organized. The mesonephric glomerulus vasculature is composed of the tubule structures that carry blood or lymph in the mesonephric glomerulus. Sources: GOC:mtg_kidney_jan10